short-chain carboxylesterase activity [GO:0034338] (molecular function) Definition: Catalysis of the reaction: a carboxylic ester + H2O = an alcohol + a carboxylic anion, where the carboxylic chain has 8 or fewer carbon atoms. Relationships: is a type of carboxylic ester hydrolase activity [GO:0052689] Also known as: short-chain esterase activity, butyrate esterase activity, butyryl esterase activity, methylbutyrase activity, methylbutyrate esterase activity, monobutyrase activity, propionyl esterase activity Subtypes: acetylesterase activity [GO:0008126] Sources: GOC:jp